{
  "gene_symbol": "CDH8",
  "gene": "UniProtKB:P55286",
  "term_label": "beta-catenin binding",
  "gene_name": "Cadherin-8",
  "term_id": "GO:0008013"
}